{
  "gene_name": "DNA-directed RNA polymerase II subunit RPB7",
  "term_label": "single-stranded RNA binding",
  "gene": "UniProtKB:P62487",
  "gene_symbol": "POLR2G",
  "term_id": "GO:0003727"
}